{
  "term_label": "Unknown biological process",
  "gene_name": "Ecto-ADP-ribosyltransferase 5",
  "gene": "UniProtKB:Q96L15",
  "term_id": "UNKNOWN:0002",
  "gene_symbol": "ART5"
}